{
  "gene": "UniProtKB:Q9Y2G2",
  "term_id": "GO:0006954",
  "gene_symbol": "CARD8",
  "gene_name": "Caspase recruitment domain-containing protein 8",
  "term_label": "inflammatory response"
}